{
  "gene": "UniProtKB:Q9NV58",
  "term_id": "GO:0006511",
  "gene_name": "E3 ubiquitin-protein ligase RNF19A",
  "gene_symbol": "RNF19A",
  "term_label": "ubiquitin-dependent protein catabolic process"
}